{
  "gene_name": "Cadherin-related family member 3",
  "gene": "UniProtKB:Q6ZTQ4",
  "term_id": "GO:0034332",
  "term_label": "adherens junction organization",
  "gene_symbol": "CDHR3"
}